protein-cysteine S-arachidonoyltransferase activity [GO:0140441] (molecular function) Relationships: is a type of protein-cysteine S-acyltransferase activity [GO:0019707] References: PMID:12681491, PMID:22247542, PMID:22968831 Sources: RHEA:59748 Definition: Catalysis of the transfer of an arachidonoyl (systematic name, (5Z,8Z,11Z,14Z)-eicosatetraenoyl) group to a sulfur atom on the cysteine of a protein molecule, in the reaction: in the reaction: (5Z,8Z,11Z,14Z)-eicosatetraenoyl-CoA + L-cysteinyl-[protein] = CoA + S-(5Z,8Z,11Z,14Z-eicosatetraenoyl)-L-cysteinyl-[protein].